{
  "gene": "UniProtKB:Q8WUA4",
  "gene_name": "General transcription factor 3C polypeptide 2",
  "term_id": "GO:0006383",
  "gene_symbol": "GTF3C2",
  "term_label": "transcription by RNA polymerase III"
}